{
  "gene_symbol": "UVSSA",
  "term_id": "GO:0006283",
  "gene_name": "UV-stimulated scaffold protein A",
  "term_label": "transcription-coupled nucleotide-excision repair",
  "gene": "UniProtKB:Q2YD98"
}